{
  "gene": "UniProtKB:P60900",
  "term_label": "cytosol",
  "gene_name": "Proteasome subunit alpha type-6",
  "gene_symbol": "PSMA6",
  "term_id": "GO:0005829"
}